{
  "gene": "UniProtKB:Q8NB66",
  "gene_name": "Protein unc-13 homolog C",
  "term_id": "GO:0030672",
  "term_label": "synaptic vesicle membrane",
  "gene_symbol": "UNC13C"
}